{
  "term_label": "xenobiotic metabolic process",
  "gene": "UniProtKB:Q16696",
  "term_id": "GO:0006805",
  "gene_symbol": "CYP2A13",
  "gene_name": "Cytochrome P450 2A13"
}